{
  "gene_name": "WD repeat-containing protein 93",
  "gene": "UniProtKB:Q6P2C0",
  "term_id": "UNKNOWN:0003",
  "term_label": "Unknown cellular component",
  "gene_symbol": "WDR93"
}